{
  "term_id": "GO:0001540",
  "gene_symbol": "ITM2B",
  "term_label": "amyloid-beta binding",
  "gene": "UniProtKB:Q9Y287",
  "gene_name": "Integral membrane protein 2B"
}